{
  "gene_symbol": "CMTM1",
  "term_id": "UNKNOWN:0002",
  "term_label": "Unknown biological process",
  "gene_name": "CKLF-like MARVEL transmembrane domain-containing protein 1",
  "gene": "UniProtKB:Q8IZ96"
}